negative regulation of potassium ion transmembrane transport [GO:1901380] (biological process) Relationships: is a type of negative regulation of potassium ion transport [GO:0043267]; is a type of regulation of potassium ion transmembrane transport [GO:1901379]; is a type of negative regulation of cation transmembrane transport [GO:1904063]; negatively regulates GO:0071805 Subtypes: negative regulation of potassium ion transmembrane transporter activity [GO:1901017], GO:1903287, negative regulation of potassium ion export across plasma membrane [GO:1903765] Also known as: down regulation of potassium ion transmembrane transport, down-regulation of potassium ion transmembrane transport, downregulation of potassium ion transmembrane transport, negative regulation of potassium ion membrane transport, inhibition of potassium ion transmembrane transport Sources: GOC:BHF, GOC:TermGenie Definition: Any process that stops, prevents or reduces the frequency, rate or extent of potassium ion transmembrane transport.